{
  "gene_symbol": "POT1",
  "term_label": "G-rich strand telomeric DNA binding",
  "gene": "UniProtKB:Q9NUX5",
  "gene_name": "Protection of telomeres protein 1",
  "term_id": "GO:0098505"
}